{
  "term_label": "Unknown molecular function",
  "term_id": "UNKNOWN:0001",
  "gene": "UniProtKB:Q8N1I8",
  "gene_name": "Putative uncharacterized protein encoded by CACTIN-AS1",
  "gene_symbol": "CACTIN-AS1"
}